{
  "gene_name": "Nuclear receptor subfamily 6 group A member 1",
  "term_label": "chromatin",
  "term_id": "GO:0000785",
  "gene_symbol": "NR6A1",
  "gene": "UniProtKB:Q15406"
}